{
  "gene": "UniProtKB:A6NHQ2",
  "term_label": "Cajal body",
  "gene_symbol": "FBLL1",
  "gene_name": "rRNA_tRNA 2'-O-methyltransferase fibrillarin-like protein 1",
  "term_id": "GO:0015030"
}